{
  "term_label": "endoplasmic reticulum",
  "gene_symbol": "ALG1L2",
  "term_id": "GO:0005783",
  "gene": "UniProtKB:C9J202",
  "gene_name": "Putative glycosyltransferase ALG1L2"
}